{
  "gene": "UniProtKB:Q14773",
  "gene_name": "Intercellular adhesion molecule 4",
  "term_id": "GO:0005886",
  "term_label": "plasma membrane",
  "gene_symbol": "ICAM4"
}